{
  "term_id": "UNKNOWN:0002",
  "gene": "UniProtKB:Q8TD06",
  "gene_name": "Anterior gradient protein 3",
  "gene_symbol": "AGR3",
  "term_label": "Unknown biological process"
}